protein transport by the Sec complex [GO:0043952] (biological process) Definition: The process in which unfolded proteins are transported across the cytoplasmic membrane in Gram-positive and Gram-negative bacteria by the Sec complex, in a process involving proteolytic cleavage of an N-terminal signal peptide. Note: Note that this term represents an activity and not a cellular structure. Consider also annotating to the cellular structure term 'cell envelope Sec protein transport complex ; GO:0031522'. For proteins involved in bacterial type II secretion across the outer membrane, consider annotating to 'protein secretion by the type II secretion system ; GO:0015628'. For proteins involved in Sec-complex dependent translocation into the eukaryotic endoplasmic reticulum, consider annotating to 'SRP-dependent cotranslational protein targeting to membrane, translocation ; GO:0006616'. Note that this term is used for annotation of proteins that compose the transport complex but not the proteins being transported. Sources: GOC:pamgo_curators Also known as: protein secretion by the Sec complex, protein translocation by the Sec complex Relationships: is a type of protein transmembrane transport [GO:0071806]